{
  "gene_symbol": "HLA-DQA2",
  "term_id": "GO:0042605",
  "term_label": "peptide antigen binding",
  "gene_name": "HLA class II histocompatibility antigen, DQ alpha 2 chain",
  "gene": "UniProtKB:P01906"
}